{
  "gene": "UniProtKB:Q8IXQ5",
  "gene_symbol": "KLHL7",
  "gene_name": "Kelch-like protein 7",
  "term_label": "Cul3-RING ubiquitin ligase complex",
  "term_id": "GO:0031463"
}